histone H4 acetyltransferase activity [GO:0010485] (molecular function) Definition: Catalysis of the reaction: acetyl-CoA + histone H4 = CoA + acetyl-histone H4. References: PMID:19056256 Also known as: H4 histone acetylase activity, H4 histone acetyltransferase activity Relationships: is a type of histone acetyltransferase activity [GO:0004402] Subtypes: GO:0043995, GO:0043996, histone H4K12 acetyltransferase activity [GO:0043997], GO:0046972